{
  "gene_symbol": "HORMAD1",
  "term_id": "GO:0000795",
  "gene_name": "HORMA domain-containing protein 1",
  "term_label": "synaptonemal complex",
  "gene": "UniProtKB:Q86X24"
}